lignin network [GO:0048224] (cellular component) Relationships: is_a cellular anatomical structure [GO:0110165]; is part of secondary cell wall [GO:0009531] Definition: An extracellular matrix part that consists of lignin in the form of a three-dimensional polymeric network. Lignins are complex racemic aromatic heteropolymers derived from a variety of phenylpropane monomers coupled together by an assortment of carbon-carbon and ether linkages. Lignin is crucial for structural integrity of the cell wall and stiffness and strength of the stem. In addition, lignin waterproofs the cell wall, enabling transport of water and solutes through the vascular system, and plays a role in protecting plants against pathogens. References: PMID:14503002, PMID:16662709 Sources: GOC:jid, GOC:mah